{
  "gene_symbol": "APC2",
  "term_label": "pattern specification process",
  "term_id": "GO:0007389",
  "gene": "UniProtKB:O95996",
  "gene_name": "Adenomatous polyposis coli protein 2"
}